{
  "term_id": "GO:0005886",
  "gene_name": "Band 4.1-like protein 3",
  "gene": "UniProtKB:Q9Y2J2",
  "gene_symbol": "EPB41L3",
  "term_label": "plasma membrane"
}